{
  "gene": "UniProtKB:Q8NEG5",
  "gene_symbol": "ZSWIM2",
  "gene_name": "E3 ubiquitin-protein ligase ZSWIM2",
  "term_label": "Unknown biological process",
  "term_id": "UNKNOWN:0002"
}